protein targeting to vacuole involved in autophagy [GO:0071211] (biological process) Definition: The process of directing proteins towards the vacuole using signals contained within the protein, occurring as part of autophagy, the process in which cells digest parts of their own cytoplasm. Regulation: regulated by regulation of protein targeting to vacuole involved in autophagy [GO:1904051]; negatively regulated by negative regulation of protein targeting to vacuole involved in autophagy [GO:1904052]; positively regulated by GO:1904053 Sources: GOC:mah Relationships: is_a GO:0006623; is part of autophagy [GO:0006914] Also known as: protein targeting to autophagosome Subtypes: protein targeting to lysosome involved in chaperone-mediated autophagy [GO:0061740]